{
  "term_label": "metalloendopeptidase activity",
  "gene_symbol": "SPG7",
  "gene_name": "Paraplegin",
  "term_id": "GO:0004222",
  "gene": "UniProtKB:Q9UQ90"
}